{
  "term_label": "Unknown molecular function",
  "gene": "UniProtKB:Q8N8R5",
  "gene_symbol": "C2orf69",
  "gene_name": "Mitochondrial protein C2orf69",
  "term_id": "UNKNOWN:0001"
}